{
  "gene": "UniProtKB:Q8TDX5",
  "term_id": "GO:0005829",
  "gene_name": "2-amino-3-carboxymuconate-6-semialdehyde decarboxylase",
  "term_label": "cytosol",
  "gene_symbol": "ACMSD"
}